prenylcysteine biosynthetic process [GO:0046311] (biological process) Definition: The chemical reactions and pathways resulting in the formation of prenylcysteine, 3-methyl-2-buten-1-yl-cysteine, a derivative of the amino acid cysteine formed by the covalent addition of a prenyl residue. Relationships: is a type of GO:0042398 Sources: GOC:ai Also known as: prenylcysteine anabolism, prenylcysteine biosynthesis, prenylcysteine formation, prenylcysteine synthesis